tRNA 3'-terminal CCA addition [GO:0001680] (biological process) Definition: Post-transcriptional addition of the terminal 3' CCA sequence to a tRNA which does not encode this sequence within the primary transcript. CCA addition proceeds by the sequential addition of CTP, CTP, and then ATP to the 3' end of the tRNA, yielding a diphosphate with each nucleotide addition. References: PMID:2247609 Sources: GOC:go_curators Relationships: is a type of GO:0042780; has part CCA tRNA nucleotidyltransferase activity [GO:0004810]; has part CC tRNA cytidylyltransferase activity [GO:0052927]; BFO_0000051 GO:0052929